{
  "term_label": "extracellular space",
  "gene_symbol": "NPPB",
  "term_id": "GO:0005615",
  "gene": "UniProtKB:P16860",
  "gene_name": "Natriuretic peptides B"
}